lymph gland crystal cell differentiation [GO:0035170] (biological process) Sources: GOC:bf, http://sdb.bio.purdue.edu/fly/gene/serpent3.htm Relationships: is a type of larval lymph gland hemocyte differentiation [GO:0035168]; is a type of GO:0042688 Definition: The process in which a relatively unspecialized larval lymph gland-derived hemocyte precursor cell acquires the specialized features of a crystal cell. Crystal cells are a class of cells that contain crystalline inclusions and are involved in the melanization of pathogenic material in the hemolymph.